{
  "gene_symbol": "IGLV1-40",
  "gene_name": "Immunoglobulin lambda variable 1-40",
  "gene": "UniProtKB:P01703",
  "term_id": "GO:0006955",
  "term_label": "immune response"
}